{
  "gene_symbol": "WDR1",
  "gene_name": "WD repeat-containing protein 1",
  "gene": "UniProtKB:O75083",
  "term_label": "actin filament depolymerization",
  "term_id": "GO:0030042"
}